{
  "gene_symbol": "KPNA1",
  "term_label": "NLS-dependent protein nuclear import complex",
  "gene": "UniProtKB:P52294",
  "gene_name": "Importin subunit alpha-5",
  "term_id": "GO:0042564"
}